{
  "term_id": "GO:0006749",
  "gene_symbol": "GSTA1",
  "term_label": "glutathione metabolic process",
  "gene_name": "Glutathione S-transferase A1",
  "gene": "UniProtKB:P08263"
}